{
  "term_id": "GO:0005158",
  "gene_name": "Insulin receptor substrate 1",
  "gene": "UniProtKB:P35568",
  "term_label": "insulin receptor binding",
  "gene_symbol": "IRS1"
}